{
  "term_label": "regulation of transcription by RNA polymerase II",
  "term_id": "GO:0006357",
  "gene_symbol": "NPAS1",
  "gene_name": "Neuronal PAS domain-containing protein 1",
  "gene": "UniProtKB:Q99742"
}